resolution of meiotic recombination intermediates [GO:0000712] (biological process) Also known as: resolution of meiotic joint molecules as recombinants Relationships: is a type of GO:0061982; BFO_0000050 reciprocal meiotic recombination [GO:0007131] References: PMID:11733053 Sources: GOC:elh Definition: The cleavage and rejoining of intermediates, such as Holliday junctions, formed during meiotic recombination to produce two intact molecules in which genetic material has been exchanged.